NuA4 histone acetyltransferase complex [GO:0035267] (cellular component) References: PMID:10966108, PMID:14966270 Sources: GOC:ecd Relationships: is a type of GO:0043189 Definition: A complex having histone acetylase activity on chromatin, as well as ATPase, DNA helicase and structural DNA binding activities. The complex is thought to be involved in double-strand DNA break repair. Subunits of the human complex include HTATIP/TIP60, TRRAP, RUVBL1, BUVBL2, beta-actin and BAF53/ACTL6A. In yeast, the complex has 13 subunits, including the catalytic subunit Esa1 (homologous to human Tip60). Also known as: TIP60 histone acetylase complex, TIP60 histone acetyltransferase complex